protein-phosphocysteine-mannosylglycerate-phosphotransferase system transporter activity [GO:0090581] (molecular function) References: PMID:14645248 Relationships: is_a protein-phosphocysteine-sugar phosphotransferase activity [GO:0090563] Definition: Catalysis of the PEP-dependent, phosphoryl transfer-driven transport of substances across a membrane. The transport happens by catalysis of the reaction: protein S-phosphocysteine + mannosylglycerate(out) = protein cysteine + mannosylglycerate phosphate(in).